{
  "gene": "UniProtKB:Q8N5B7",
  "term_id": "GO:0046513",
  "term_label": "ceramide biosynthetic process",
  "gene_name": "Ceramide synthase 5",
  "gene_symbol": "CERS5"
}